{
  "gene": "UniProtKB:Q96JK4",
  "term_id": "UNKNOWN:0001",
  "term_label": "Unknown molecular function",
  "gene_symbol": "HHIPL1",
  "gene_name": "HHIP-like protein 1"
}